{
  "term_label": "glucose-6-phosphate transport",
  "term_id": "GO:0015760",
  "gene_name": "Glucose-6-phosphate exchanger SLC37A4",
  "gene_symbol": "SLC37A4",
  "gene": "UniProtKB:O43826"
}